adhesion of symbiont infection structure to host [GO:0075001] (biological process) Note: Note that this term should not be used to annotate gene products of the host. It should only be used to annotate those gene products of the symbiont involved in this process. Sources: GOC:pamgo_curators Also known as: adhesion of symbiont infection structure to host during symbiotic interaction, attachment of symbiont infection structure to host Subtypes: adhesion of symbiont germination tube to host [GO:0075002], GO:0075003, adhesion of symbiont infection cushion to host [GO:0075069], adhesion of symbiont hyphopodium to host [GO:0075070], adhesion of symbiont haustorium mother cell to host [GO:0075196] Definition: The attachment of an infection structure of the symbiont to its host via adhesion molecules, general stickiness etc., either directly or indirectly. The host is defined as the larger of the organisms involved in a symbiotic interaction. Relationships: is a type of adhesion of symbiont to host [GO:0044406]